{
  "gene_name": "DNA-directed RNA polymerase II subunit RPB11-b1",
  "gene_symbol": "POLR2J2",
  "term_label": "DNA-directed RNA polymerase activity",
  "term_id": "GO:0003899",
  "gene": "UniProtKB:Q9GZM3"
}